{
  "gene_name": "N-acetylaspartylglutamate synthase A",
  "term_label": "N-acetyl-L-aspartate-L-glutamate ligase activity",
  "gene": "UniProtKB:Q8IXN7",
  "term_id": "GO:0072590",
  "gene_symbol": "RIMKLA"
}